{
  "gene": "UniProtKB:Q14746",
  "gene_symbol": "COG2",
  "gene_name": "Conserved oligomeric Golgi complex subunit 2",
  "term_label": "Golgi transport complex",
  "term_id": "GO:0017119"
}